host cell late endosome membrane [GO:0044185] (cellular component) Definition: The lipid bilayer surrounding a host cell late endosome. Sources: GOC:jl Relationships: is a type of host cell endosome membrane [GO:0044175]; is part of host cell late endosome [GO:0044184]